{
  "term_label": "chemokine (C-C motif) ligand 5 binding",
  "gene": "UniProtKB:P32246",
  "term_id": "GO:0071791",
  "gene_name": "C-C chemokine receptor type 1",
  "gene_symbol": "CCR1"
}